phosphatidylcholine binding [GO:0031210] (molecular function) Relationships: is a type of phospholipid binding [GO:0005543]; is a type of cation binding [GO:0043169]; is a type of quaternary ammonium group binding [GO:0050997] Definition: Binding to a phosphatidylcholine, a glycophospholipid in which a phosphatidyl group is esterified to the hydroxyl group of choline. Sources: GOC:mah, ISBN:0198506732